immunoglobulin binding [GO:0019865] (molecular function) Sources: GOC:ma Subtypes: polymeric immunoglobulin binding [GO:0001790], IgM binding [GO:0001791], IgA binding [GO:0019862], IgE binding [GO:0019863], IgG binding [GO:0019864], GO:0043472 Relationships: is a type of protein-containing complex binding [GO:0044877] Definition: Binding to an immunoglobulin.